{
  "gene_symbol": "KIF21B",
  "term_label": "cytoplasm",
  "gene_name": "Kinesin-like protein KIF21B",
  "gene": "UniProtKB:O75037",
  "term_id": "GO:0005737"
}